{
  "term_id": "GO:0005783",
  "gene_name": "Transmembrane emp24 domain-containing protein 6",
  "gene": "UniProtKB:Q8WW62",
  "term_label": "endoplasmic reticulum",
  "gene_symbol": "TMED6"
}